regulation of adult chitin-containing cuticle pigmentation [GO:0048082] (biological process) Definition: Any process that modulates the frequency, rate or extent of establishment of the adult pattern of pigmentation in the cuticle of an organism. Sources: GOC:jid, GOC:mtg_sensu Relationships: is a type of regulation of cuticle pigmentation [GO:0048079]; regulates adult chitin-containing cuticle pigmentation [GO:0048085] Subtypes: GO:0048083, GO:0048084